protein localization to cell division site involved in mitotic actomyosin contractile ring assembly [GO:1903476] (biological process) Regulation: regulated by GO:0110082; positively regulated by positive regulation of protein localization to cell division site involved in mitotic actomyosin contractile ring assembly [GO:0110083]; RO_0002212 by negative regulation of protein localization to cell division site involved in mitotic actomyosin contractile ring assembly [GO:0110084] Also known as: protein localisation to cell division site involved in mitotic actomyosin contractile ring assembly, protein localization to cell division site involved in actomyosin contractile ring assembly involved in cytokinesis after mitosis, protein localization to cell division site involved in contractile ring assembly involved in mitotic cytokinesis Sources: GOC:TermGenie, GOC:mtg_cell_cycle, GO_REF:0000060 Definition: Any protein localization to cell division site that is involved in mitotic actomyosin contractile ring assembly. Relationships: is_a protein localization to cell division site involved in cytokinesis, actomyosin contractile ring assembly [GO:1902575]; is part of GO:1903475